{
  "term_id": "GO:0031011",
  "gene": "UniProtKB:Q6PI98",
  "term_label": "Ino80 complex",
  "gene_name": "INO80 complex subunit C",
  "gene_symbol": "INO80C"
}